vascular endothelial growth factor receptor 1 binding [GO:0043183] (molecular function) Also known as: Flt-1 binding, VEGF receptor 1 binding, VEGFR 1 binding Sources: GOC:st Relationships: is a type of vascular endothelial growth factor receptor binding [GO:0005172] Definition: Binding to a vascular endothelial growth factor receptor 1.